{
  "gene_symbol": "A0A6Q8PHS2",
  "term_label": "Unknown molecular function",
  "gene_name": "Uncharacterized protein",
  "term_id": "UNKNOWN:0001",
  "gene": "UniProtKB:A0A6Q8PHS2"
}